{
  "term_id": "UNKNOWN:0001",
  "gene": "UniProtKB:Q8N4S9",
  "gene_name": "MARVEL domain-containing protein 2",
  "term_label": "Unknown molecular function",
  "gene_symbol": "MARVELD2"
}